Lewis x epitope biosynthetic process [GO:0106402] (biological process) References: PMID:16973732, PMID:23000574 Also known as: sLeX biosynthetic process, sialyl-Lewis X biosynthetic process Relationships: is a type of carbohydrate derivative biosynthetic process [GO:1901137] Definition: The chemical reactions and pathways resulting in the formation of a Lewis x epitope, a trisaccharide (beta-D-galactosyl-(1,4)-[alpha-L-fucosyl-(1,3)]-N-acetyl-beta-D-glucosamine) expressed on several glycolipids, glycoproteins, and proteoglycans of the nervous system. The related Lewis x epitope is formed by alpha(1,3) fucosylation of the N-acetylglucosaminyl residue of a type 2 histo-blood group antigen precursor disaccharide.